{
  "term_id": "GO:1990756",
  "gene_symbol": "KLHL5",
  "term_label": "ubiquitin-like ligase-substrate adaptor activity",
  "gene": "UniProtKB:Q96PQ7",
  "gene_name": "Kelch-like protein 5"
}